{
  "gene": "UniProtKB:P49747",
  "gene_symbol": "COMP",
  "gene_name": "Cartilage oligomeric matrix protein",
  "term_id": "UNKNOWN:0001",
  "term_label": "Unknown molecular function"
}